tRNA cytidine N4-acetyltransferase activity [GO:0051392] (molecular function) Definition: Catalysis of the reaction: a cytidine in tRNA + acetyl-CoA + ATP + H2O = ADP + an N4-acetylcytidine in tRNA + CoA + H+ + phosphate. Also known as: tRNA N4-acetyltransferase activity Relationships: is a type of GO:0008080; is a type of catalytic activity, acting on a tRNA [GO:0140101] References: PMID:15037780 Sources: RHEA:53876